{
  "term_label": "Unknown molecular function",
  "gene_symbol": "DTHD1",
  "gene": "UniProtKB:Q6ZMT9",
  "term_id": "UNKNOWN:0001",
  "gene_name": "Death domain-containing protein 1"
}